{
  "gene_symbol": "KLHL10",
  "term_id": "GO:0043161",
  "term_label": "proteasome-mediated ubiquitin-dependent protein catabolic process",
  "gene": "UniProtKB:Q6JEL2",
  "gene_name": "Kelch-like protein 10"
}